cytochrome-c oxidase activity [GO:0004129] (molecular function) Regulation: regulated by regulation of cytochrome-c oxidase activity [GO:1904959]; positively regulated by positive regulation of cytochrome-c oxidase activity [GO:1904960] Definition: Catalysis of the reaction: 4 Fe(II)-[cytochrome c] + O2 + 8 H+(in) = 4 Fe(III)-[cytochrome c] + 2 H2O + 4 H+(out). Relationships: is_a GO:0009055; is a type of GO:0015078; is a type of oxidoreduction-driven active transmembrane transporter activity [GO:0015453]; is a type of active monoatomic ion transmembrane transporter activity [GO:0022853]; has part oxidoreductase activity, acting on a heme group of donors [GO:0016675] Note: The reduction of O2 to water is accompanied by the extrusion of four protons from the intramitochondrial compartment. Sources: RHEA:11436 Also known as: cytochrome c oxidase activity, aa3-type cytochrome c oxidase, ba3-type cytochrome c oxidase, caa3-type cytochrome c oxidase, cbb3-type cytochrome c oxidase, cytochrome a3 activity, cytochrome aa3 activity, indophenol oxidase, indophenolase, Warburg's respiratory enzyme activity, complex IV (mitochondrial electron transport) activity, cytochrome oxidase activity